hematopoietic stem cell migration [GO:0035701] (biological process) Definition: The orderly movement of a hematopoietic stem cell from one site to another. A hematopoietic stem cell is a cell from which all cells of the lymphoid and myeloid lineages develop, including blood cells and cells of the immune system. References: PMID:20234092 Sources: CL:0000037, GOC:BHF Also known as: hemopoietic stem cell migration Relationships: is a type of cell migration [GO:0016477] Subtypes: GO:0097241 Regulation: regulated by regulation of hematopoietic stem cell migration [GO:2000471]; negatively regulated by negative regulation of hematopoietic stem cell migration [GO:2000472]; positively regulated by GO:2000473